{
  "gene": "UniProtKB:Q9H672",
  "term_label": "Unknown biological process",
  "gene_name": "Ankyrin repeat and SOCS box protein 7",
  "gene_symbol": "ASB7",
  "term_id": "UNKNOWN:0002"
}